NAD(P)H dehydrogenase complex assembly [GO:0010275] (biological process) Subtypes: NADH dehydrogenase complex (plastoquinone) assembly [GO:0010258] Sources: GOC:sm Also known as: NAD(P)H dehydrogenase complex (plastoquinone) assembly Relationships: is a type of protein-containing complex assembly [GO:0065003] Definition: The aggregation, arrangement and bonding together of a set of components to form NAD(P)H dehydrogenase complex, which is involved in electron transport from an unidentified electron donor, possibly NAD(P)H or ferredoxin(Fd) to the plastoquinone pool.